{
  "gene": "UniProtKB:Q5T5P2",
  "term_id": "UNKNOWN:0002",
  "gene_symbol": "KIAA1217",
  "term_label": "Unknown biological process",
  "gene_name": "Sickle tail protein homolog"
}